2-polyprenyl-6-hydroxyphenol methylase activity [GO:0102208] (molecular function) Relationships: is a type of methyltransferase activity [GO:0008168] Definition: Catalysis of the reaction: a 3-(all-trans-polyprenyl)benzene-1,2-diol + S-adenosyl-L-methionine = a 2-methoxy-6-(all-trans-polyprenyl)phenol + H+ + S-adenosyl-L-homocysteine. Sources: GOC:pz, RHEA:31411